{
  "gene": "UniProtKB:Q01201",
  "term_id": "GO:0006954",
  "term_label": "inflammatory response",
  "gene_symbol": "RELB",
  "gene_name": "Transcription factor RelB"
}